L-serine transport [GO:0015825] (biological process) Subtypes: L-serine transmembrane import into vacuole [GO:0090516], L-serine import across plasma membrane [GO:1903812] Sources: GOC:ai, GOC:jsg, GOC:mah Definition: The directed movement of L-serine, the L-enantiomer of 2-amino-3-hydroxypropanoic acid, into, out of or within a cell, or between cells, by means of some agent such as a transporter or pore. Relationships: is a type of L-amino acid transport [GO:0015807]; is a type of serine transport [GO:0032329] Also known as: L-serine import